{
  "gene_symbol": "THY1",
  "gene_name": "Thy-1 membrane glycoprotein",
  "gene": "UniProtKB:P04216",
  "term_id": "GO:0005096",
  "term_label": "GTPase activator activity"
}